serotonin production involved in inflammatory response [GO:0002351] (biological process) Also known as: serotonin production involved in acute inflammatory response References: PMID:16730260 Sources: GOC:add, ISBN:0781735149 Definition: The synthesis or release of serotonin following a stimulus as part of an inflammatory response, resulting in an increase in its intracellular or extracellular levels. Relationships: is a type of production of molecular mediator involved in inflammatory response [GO:0002532]